vasomotion [GO:1990029] (BP) Definition: The rhythmical contraction and relaxation of arterioles, observed as slow and fast waves, with frequencies of 1-2 and 10-20 cpm. References: PMID:14993429, PMID:15678091, PMID:1932763 Sources: GOC:sl Relationships: is a type of circulatory system process [GO:0003013]